{
  "gene_name": "Electrogenic sodium bicarbonate cotransporter 1",
  "gene_symbol": "SLC4A4",
  "term_id": "GO:0015701",
  "gene": "UniProtKB:Q9Y6R1",
  "term_label": "bicarbonate transport"
}